microsporocyte nucleus [GO:0048556] (CC) Relationships: is a type of nucleus [GO:0005634] Sources: GOC:tair_curators, ISBN:047186840X Also known as: microspore mother cell nucleus, pollen mother cell nucleus Definition: The nucleus of the microsporocyte. The microsporocyte is a diploid cell in which meiosis will occur, resulting in four microspores. A microspore is a spore that, in vascular plants, gives rise to a male gametophyte.